negative regulation of galactotriose transport [GO:1900292] (biological process) Sources: GOC:TermGenie, GOC:mengo_curators Definition: Any process that stops, prevents or reduces the frequency, rate or extent of galactotriose transport. Relationships: is_a GO:0051051; is a type of GO:1900291; negatively regulates GO:2001093 Also known as: down regulation of galactotriose transport, down-regulation of galactotriose transport, downregulation of galactotriose transport, inhibition of galactotriose transport